indolepyruvate decarboxylase activity [GO:0047434] (molecular function) Relationships: is a type of GO:0016831 Definition: Catalysis of the reaction: indolepyruvate = CO2 + indole acetaldehyde. Also known as: 3-(indol-3-yl)pyruvate carboxy-lyase [(2-indol-3-yl)acetaldehyde-forming], 3-(indol-3-yl)pyruvate carboxy-lyase activity, indol-3-yl-pyruvate carboxy-lyase activity, indole-3-pyruvate decarboxylase activity Sources: EC:4.1.1.74, MetaCyc:4.1.1.74-RXN